{
  "gene_symbol": "PPP1CB",
  "gene_name": "Serine_threonine-protein phosphatase PP1-beta catalytic subunit",
  "gene": "UniProtKB:P62140",
  "term_label": "regulation of circadian rhythm",
  "term_id": "GO:0042752"
}